MICOS complex [GO:0061617] (CC) Definition: Mitochondrial inner membrane complex involved in maintenance of crista junctions, inner membrane architecture, and formation of contact sites to the outer membrane. In Saccharomyces cerevisiae the complex has six subunits: MIC10, MIC12, MIC19, MIC26, MIC27, and MIC60. References: PMID:21944719, PMID:21987634, PMID:22009199, PMID:24687277 Sources: GOC:dph Also known as: Fcj1 complex, MINOS complex, MitOS complex, mitochondrial contact site and cristae organizing system Relationships: is a type of GO:0098800